{
  "term_id": "UNKNOWN:0002",
  "term_label": "Unknown biological process",
  "gene_symbol": "DDX27",
  "gene_name": "Probable ATP-dependent RNA helicase DDX27",
  "gene": "UniProtKB:Q96GQ7"
}